{
  "term_label": "signal transduction",
  "gene_name": "Growth factor receptor-bound protein 2",
  "term_id": "GO:0007165",
  "gene": "UniProtKB:P62993",
  "gene_symbol": "GRB2"
}